{
  "gene_symbol": "RPP38-DT",
  "gene": "UniProtKB:Q8N326",
  "term_label": "Unknown biological process",
  "term_id": "UNKNOWN:0002",
  "gene_name": "Putative uncharacterized protein RPP38-DT"
}